{
  "gene_name": "Beta-1,4-galactosyltransferase 7",
  "term_id": "GO:0005794",
  "term_label": "Golgi apparatus",
  "gene_symbol": "B4GALT7",
  "gene": "UniProtKB:Q9UBV7"
}